{
  "gene": "UniProtKB:P52803",
  "gene_name": "Ephrin-A5",
  "term_id": "GO:0007411",
  "gene_symbol": "EFNA5",
  "term_label": "axon guidance"
}